negative regulation of interleukin-2-mediated signaling pathway [GO:1902206] (biological process) References: PMID:11909529 Sources: GOC:TermGenie Definition: Any process that stops, prevents or reduces the frequency, rate or extent of interleukin-2-mediated signaling pathway. Also known as: down regulation of IL-2-mediated signaling pathway, down regulation of interleukin-2-mediated signaling pathway, down regulation of interleukin-2-mediated signalling pathway, down-regulation of IL-2-mediated signaling pathway, down-regulation of interleukin-2-mediated signaling pathway, down-regulation of interleukin-2-mediated signalling pathway, downregulation of IL-2-mediated signaling pathway, downregulation of interleukin-2-mediated signaling pathway, downregulation of interleukin-2-mediated signalling pathway, negative regulation of IL-2-mediated signaling pathway, negative regulation of interleukin-2-mediated signalling pathway, inhibition of IL-2-mediated signaling pathway, inhibition of interleukin-2-mediated signaling pathway, inhibition of interleukin-2-mediated signalling pathway Relationships: is a type of GO:0001960; is a type of GO:1902205; RO_0002212 interleukin-2-mediated signaling pathway [GO:0038110]